{
  "gene_name": "Dolichyl pyrophosphate Man9GlcNAc2 alpha-1,3-glucosyltransferase",
  "term_id": "GO:0006488",
  "gene": "UniProtKB:Q9Y672",
  "gene_symbol": "ALG6",
  "term_label": "dolichol-linked oligosaccharide biosynthetic process"
}